mesonephric renal vesicle formation [GO:0061262] (biological process) Regulation: positively regulated by mesonephric renal vesicle induction [GO:0061294] Sources: GOC:mtg_kidney_jan10 Definition: The developmental process pertaining to the initial formation of the mesonephros. Also known as: mesonephros formation Relationships: is a type of renal vesicle formation [GO:0072033]; is part of mesonephric renal vesicle morphogenesis [GO:0061243]